{
  "term_label": "Unknown cellular component",
  "gene": "UniProtKB:Q8NES8",
  "gene_symbol": "DEFB124",
  "term_id": "UNKNOWN:0003",
  "gene_name": "Beta-defensin 124"
}